{
  "term_label": "Unknown molecular function",
  "gene_symbol": "DANCR",
  "gene_name": "Putative uncharacterized protein DANCR",
  "gene": "UniProtKB:P0C864",
  "term_id": "UNKNOWN:0001"
}